{
  "gene": "UniProtKB:Q13131",
  "gene_name": "5'-AMP-activated protein kinase catalytic subunit alpha-1",
  "term_label": "protein localization to lipid droplet",
  "gene_symbol": "PRKAA1",
  "term_id": "GO:1990044"
}